{
  "gene_symbol": "MGST2",
  "term_id": "GO:0004464",
  "term_label": "leukotriene-C4 synthase activity",
  "gene_name": "Microsomal glutathione S-transferase 2",
  "gene": "UniProtKB:Q99735"
}